{
  "gene_name": "C-C motif chemokine 15",
  "term_label": "inflammatory response",
  "gene_symbol": "CCL15",
  "gene": "UniProtKB:Q16663",
  "term_id": "GO:0006954"
}